R2TP complex [GO:0097255] (cellular component) References: PMID:15766533, PMID:21925213 Sources: GOC:mcc Relationships: is a type of protein-containing complex [GO:0032991] Definition: A highly conserved protein complex comprised of two ATP-dependent DNA helicases (Rvb1p and Rvb2p in yeast, Pontin52 and Reptin52 in humans), Pih1p in yeast or PIH1D1 in humans, and Tah1 in yeast or RPAP3 in humans. The complex associates with Hsp90 and is thought to have a role in assembly of large protein or protein/nucleic acid complexes. In this role it is involved in multiple processes such as box C/D snoRNP biogenesis, phosphatidylinositol-3 kinase-related protein kinase (PIKK) signaling, RNA polymerase II assembly, and others.